{
  "gene_name": "Small ubiquitin-related modifier 5",
  "gene": "UniProtKB:G2XKQ0",
  "term_id": "GO:0016605",
  "gene_symbol": "SUMO1P1",
  "term_label": "PML body"
}